{
  "gene_symbol": "YBX2",
  "gene_name": "Y-box-binding protein 2",
  "gene": "UniProtKB:Q9Y2T7",
  "term_label": "regulation of gene expression",
  "term_id": "GO:0010468"
}